{
  "gene_symbol": "RAMP2",
  "term_id": "GO:0006816",
  "term_label": "calcium ion transport",
  "gene_name": "Receptor activity-modifying protein 2",
  "gene": "UniProtKB:O60895"
}